{
  "gene": "UniProtKB:P45379",
  "term_label": "sarcomere organization",
  "gene_symbol": "TNNT2",
  "gene_name": "Troponin T, cardiac muscle",
  "term_id": "GO:0045214"
}